D-ribose transmembrane transport [GO:0015752] (biological process) Definition: The process in which D-ribose is transported across a lipid bilayer, from one side of a membrane to the other. As beta-D-ribofuranose, D-ribose forms the glycose group of all ribonucleosides, ribonucleotides and ribonucleic acids, and also of ribose phosphates, various glycosides, some coenzymes and some forms of vitamin B12. Relationships: is a type of GO:0015750 Sources: GOC:ai Also known as: D-ribose transport